{
  "term_label": "cytoplasm",
  "term_id": "GO:0005737",
  "gene": "UniProtKB:Q96DT0",
  "gene_name": "Galectin-12",
  "gene_symbol": "LGALS12"
}